sieve element enucleation [GO:0090602] (biological process) Relationships: is a type of enucleation [GO:0090601]; is part of sieve element differentiation [GO:0090603] References: PMID:25081480 Sources: GOC:tb Definition: The process in which nucleated precursor cells lose their nucleus as part of sieve element differentiation. The nuclear contents are released and degraded in the cytoplasm at the same time as other organelles are rearranged and the cytosol is degraded.